{
  "term_label": "regulation of proteolysis",
  "gene": "UniProtKB:O43791",
  "gene_symbol": "SPOP",
  "term_id": "GO:0030162",
  "gene_name": "Speckle-type POZ protein"
}